{
  "term_label": "immune system process",
  "gene_name": "Interferon regulatory factor 6",
  "gene": "UniProtKB:O14896",
  "gene_symbol": "IRF6",
  "term_id": "GO:0002376"
}